{
  "term_id": "GO:0005109",
  "term_label": "frizzled binding",
  "gene_name": "Protein Wnt-4",
  "gene_symbol": "WNT4",
  "gene": "UniProtKB:P56705"
}